{
  "term_id": "GO:0000981",
  "term_label": "DNA-binding transcription factor activity, RNA polymerase II-specific",
  "gene_symbol": "GZF1",
  "gene_name": "GDNF-inducible zinc finger protein 1",
  "gene": "UniProtKB:Q9H116"
}